{
  "term_id": "GO:0004407",
  "term_label": "histone deacetylase activity",
  "gene_symbol": "HDAC2",
  "gene": "UniProtKB:Q92769",
  "gene_name": "Histone deacetylase 2"
}